sialate 9-O-acetylesterase activity [GO:0106330] (molecular function) Relationships: is_a sialate O-acetylesterase activity [GO:0001681] References: PMID:22291594 Sources: RHEA:22600 Definition: Catalysis of the reaction: H2O + N-acetyl-9-O-acetylneuraminate = acetate + H+ + N-acetylneuraminate.